{
  "gene_symbol": "CSH1",
  "gene": "UniProtKB:P0DML2",
  "term_label": "growth hormone receptor binding",
  "term_id": "GO:0005131",
  "gene_name": "Chorionic somatomammotropin hormone 1"
}